{
  "gene_symbol": "ZNF792",
  "gene": "UniProtKB:Q3KQV3",
  "term_id": "GO:0006357",
  "term_label": "regulation of transcription by RNA polymerase II",
  "gene_name": "Zinc finger protein 792"
}